{
  "gene_symbol": "C5orf64",
  "term_id": "UNKNOWN:0003",
  "term_label": "Unknown cellular component",
  "gene": "UniProtKB:Q2M2E5",
  "gene_name": "Uncharacterized protein C5orf64"
}